{
  "gene_symbol": "ADRA2A",
  "term_label": "epinephrine binding",
  "gene_name": "Alpha-2A adrenergic receptor",
  "gene": "UniProtKB:P08913",
  "term_id": "GO:0051379"
}